{
  "gene": "UniProtKB:Q9NWN3",
  "gene_symbol": "FBXO34",
  "term_id": "UNKNOWN:0002",
  "gene_name": "F-box only protein 34",
  "term_label": "Unknown biological process"
}